{
  "term_id": "GO:0034451",
  "term_label": "centriolar satellite",
  "gene_symbol": "ZMYND10",
  "gene": "UniProtKB:O75800",
  "gene_name": "Zinc finger MYND domain-containing protein 10"
}